granaticin catabolic process [GO:1901108] (biological process) Relationships: is a type of GO:0030640; is a type of ketone catabolic process [GO:0042182] Definition: The chemical reactions and pathways resulting in the breakdown of granaticin. Sources: GOC:TermGenie, GOC:yaf, UniPathway:UPA00175 Also known as: granaticin breakdown, granaticin catabolism, granaticin degradation